{
  "gene": "UniProtKB:P49720",
  "gene_symbol": "PSMB3",
  "gene_name": "Proteasome subunit beta type-3",
  "term_id": "GO:0019774",
  "term_label": "proteasome core complex, beta-subunit complex"
}